sensory organ morphogenesis [GO:0090596] (biological process) Sources: GOC:kmv, ISBN:978-0199210893 Definition: Morphogenesis of a sensory organ. A sensory organ is defined as a tissue or set of tissues that work together to receive and transmit signals from external or internal stimuli. Morphogenesis is the process in which anatomical structures are generated and organized. Organs are commonly observed as visibly distinct structures, but may also exist as loosely associated clusters of cells that work together to perform a specific function or functions. Subtypes: ear morphogenesis [GO:0042471], GO:0043585, tongue morphogenesis [GO:0043587], eye morphogenesis [GO:0048592], ocellus morphogenesis [GO:0048816], taste bud morphogenesis [GO:0061194], nematode male tail mating organ morphogenesis [GO:0090597] Relationships: is a type of animal organ morphogenesis [GO:0009887]; is part of sensory organ development [GO:0007423]